{
  "term_label": "Unknown molecular function",
  "gene": "UniProtKB:Q8WV99",
  "term_id": "UNKNOWN:0001",
  "gene_name": "AN1-type zinc finger protein 2B",
  "gene_symbol": "ZFAND2B"
}